{
  "term_label": "regulation of transcription by RNA polymerase II",
  "gene": "UniProtKB:P36956",
  "term_id": "GO:0006357",
  "gene_symbol": "SREBF1",
  "gene_name": "Sterol regulatory element-binding protein 1"
}